inositol-1,3,4,5,6-pentakisphosphate 1-phosphatase activity [GO:0052825] (molecular function) Definition: Catalysis of the reaction: inositol-1,3,4,5,6-pentakisphosphate + H2O = inositol-3,4,5,6-tetrakisphosphate + phosphate. Relationships: is a type of GO:0052827 Sources: GOC:ai